{
  "term_id": "GO:0070822",
  "gene_symbol": "BRMS1",
  "gene_name": "Breast cancer metastasis-suppressor 1",
  "gene": "UniProtKB:Q9HCU9",
  "term_label": "Sin3-type complex"
}